metalloendopeptidase activity [GO:0004222] (molecular function) Definition: Catalysis of the hydrolysis of internal, alpha-peptide bonds in a polypeptide chain by a mechanism in which water acts as a nucleophile, one or two metal ions hold the water molecule in place, and charged amino acid side chains are ligands for the metal ions. Relationships: is a type of endopeptidase activity [GO:0004175]; is a type of metallopeptidase activity [GO:0008237] Regulation: negatively regulated by metalloendopeptidase inhibitor activity [GO:0008191]; positively regulated by GO:1904685 Subtypes: GO:1902945 Sources: GOC:mah, https://www.ebi.ac.uk/merops/about/glossary.shtml#CATTYPE, https://www.ebi.ac.uk/merops/about/glossary.shtml#ENDOPEPTIDASE Also known as: metalloendoprotease activity, metalloendoproteinase activity